TMP catabolic process [GO:0046045] (biological process) Also known as: TMP breakdown, TMP catabolism, TMP degradation Definition: The chemical reactions and pathways resulting in the breakdown of TMP, ribosylthymine monophosphate. Relationships: is a type of GO:0009175; is a type of GO:0009222; is a type of TMP metabolic process [GO:0046044] Sources: GOC:go_curators